{
  "term_id": "GO:0019901",
  "gene_symbol": "RAC3",
  "gene_name": "Ras-related C3 botulinum toxin substrate 3",
  "gene": "UniProtKB:P60763",
  "term_label": "protein kinase binding"
}